{
  "gene": "UniProtKB:P27487",
  "gene_name": "Dipeptidyl peptidase 4",
  "term_label": "plasma membrane",
  "term_id": "GO:0005886",
  "gene_symbol": "DPP4"
}